bronchus cartilage development [GO:0060532] (biological process) Relationships: is a type of GO:0051216; is part of bronchus development [GO:0060433] Sources: GOC:dph, GOC:mtg_lung Also known as: pulmonary cartilage development Definition: The process whose specific outcome is the progression of lung cartilage over time, from its formation to the mature structure. Cartilage is a connective tissue dominated by extracellular matrix containing collagen type II and large amounts of proteoglycan, particularly chondroitin sulfate.